xylan O-acetyltransferase activity [GO:1990538] (molecular function) Relationships: is a type of O-acetyltransferase activity [GO:0016413] Definition: Catalysis of the reaction: acetyl-CoA + a xylan= CoA + an acetylated xylan. References: PMID:25141999